2-deoxy-D-gluconate 3-dehydrogenase activity [GO:0008678] (molecular function) Sources: EC:1.1.1.125 Also known as: 2-deoxy-D-gluconate:NAD+ 3-oxidoreductase activity, 2-deoxygluconate dehydrogenase activity, 2-keto-3-deoxygluconate oxidoreductase activity Relationships: is a type of oxidoreductase activity, acting on the CH-OH group of donors, NAD or NADP as acceptor [GO:0016616] Definition: Catalysis of the reaction: 2-deoxy-D-gluconate + NAD+ = 3-dehydro-2-deoxy-D-gluconate + NADH + H+.